{
  "term_label": "transcription regulator complex",
  "term_id": "GO:0005667",
  "gene": "UniProtKB:A0A1W2PR48",
  "gene_name": "Transducin-like enhancer protein 7",
  "gene_symbol": "TLE7"
}